{
  "gene_symbol": "C9orf163",
  "gene_name": "Uncharacterized protein C9orf163",
  "term_id": "UNKNOWN:0001",
  "gene": "UniProtKB:Q8N9P6",
  "term_label": "Unknown molecular function"
}